{
  "term_id": "GO:0005739",
  "gene_symbol": "GTPBP10",
  "term_label": "mitochondrion",
  "gene_name": "GTP-binding protein 10",
  "gene": "UniProtKB:A4D1E9"
}